bud field specification [GO:0061139] (biological process) Definition: The regionalization process in which the identity of a bud primordium is specified. Identity is considered to be the aggregate of characteristics by which a structure is recognized. Relationships: is a type of regionalization [GO:0003002]; is part of morphogenesis of a branching epithelium [GO:0061138] Sources: GOC:dph